{
  "term_id": "GO:0007186",
  "gene_name": "Rhodopsin",
  "gene": "UniProtKB:P08100",
  "gene_symbol": "RHO",
  "term_label": "G protein-coupled receptor signaling pathway"
}